{
  "gene_name": "Probable G-protein coupled receptor 88",
  "term_id": "GO:0008020",
  "gene_symbol": "GPR88",
  "term_label": "G protein-coupled photoreceptor activity",
  "gene": "UniProtKB:Q9GZN0"
}